{
  "term_id": "GO:0030055",
  "gene_symbol": "FERMT3",
  "gene": "UniProtKB:Q86UX7",
  "term_label": "cell-substrate junction",
  "gene_name": "Fermitin family homolog 3"
}